{
  "gene": "UniProtKB:P14902",
  "term_label": "L-tryptophan catabolic process to kynurenine",
  "gene_name": "Indoleamine 2,3-dioxygenase 1",
  "gene_symbol": "IDO1",
  "term_id": "GO:0019441"
}